{
  "gene": "UniProtKB:Q8IUY3",
  "term_label": "organelle membrane contact site",
  "term_id": "GO:0044232",
  "gene_symbol": "GRAMD2A",
  "gene_name": "GRAM domain-containing protein 2A"
}